pre-B cell allelic exclusion [GO:0002331] (biological process) Relationships: is a type of GO:0010468; BFO_0000050 pre-B cell differentiation [GO:0002329] Definition: Expression of a single heavy chain allele during pre-B cell differentiation. Sources: GOC:add, GOC:jal, ISBN:0781735149 Also known as: pre-B lymphocyte allelic exclusion